{
  "gene_symbol": "TXNRD1",
  "term_id": "GO:0005829",
  "gene": "UniProtKB:Q16881",
  "gene_name": "Thioredoxin reductase 1, cytoplasmic",
  "term_label": "cytosol"
}